{
  "gene_name": "Replication factor C subunit 3",
  "term_id": "GO:0005634",
  "gene_symbol": "RFC3",
  "term_label": "nucleus",
  "gene": "UniProtKB:P40938"
}